positive regulation of spermatid nuclear differentiation [GO:0045702] (biological process) Relationships: is a type of positive regulation of organelle organization [GO:0010638]; is a type of positive regulation of cell differentiation [GO:0045597]; is_a regulation of spermatid nuclear differentiation [GO:0045700]; is a type of positive regulation of reproductive process [GO:2000243]; positively regulates GO:0007289 Also known as: up regulation of spermatid nuclear differentiation, up-regulation of spermatid nuclear differentiation, upregulation of spermatid nuclear differentiation, activation of spermatid nuclear differentiation, stimulation of spermatid nuclear differentiation Sources: GOC:go_curators Definition: Any process that activates or increases the frequency, rate or extent of spermatid nuclear differentiation.